{
  "gene_symbol": "PFKFB2",
  "term_id": "GO:0005829",
  "gene_name": "6-phosphofructo-2-kinase_fructose-2,6-bisphosphatase 2",
  "term_label": "cytosol",
  "gene": "UniProtKB:O60825"
}